{
  "gene": "UniProtKB:P15918",
  "term_id": "GO:1990238",
  "gene_symbol": "RAG1",
  "term_label": "double-stranded DNA endonuclease activity",
  "gene_name": "V(D)J recombination-activating protein 1"
}